cytostome [GO:0031910] (cellular component) References: PMID:10503189 Relationships: is a type of cellular anatomical structure [GO:0110165]; is part of GO:0005886 Definition: Stable, specialized structure for the ingestion of food by the cell into phagosomes.